protocatechuate decarboxylase activity [GO:0050223] (molecular function) Also known as: 3,4-dihydrobenzoate decarboxylase activity, 3,4-dihydroxybenzoate carboxy-lyase (catechol-forming), 3,4-dihydroxybenzoate decarboxylase activity, protocatechuate carboxy-lyase activity Sources: EC:4.1.1.63, RHEA:22416 Relationships: is a type of carboxy-lyase activity [GO:0016831] Definition: Catalysis of the reaction: 3,4-dihydroxybenzoate + H+ = catechol + CO2.